{
  "term_label": "cell adhesion mediator activity",
  "term_id": "GO:0098631",
  "gene": "UniProtKB:Q15223",
  "gene_symbol": "NECTIN1",
  "gene_name": "Nectin-1"
}